{
  "gene_symbol": "MAGOHB",
  "gene_name": "Protein mago nashi homolog 2",
  "term_id": "UNKNOWN:0001",
  "gene": "UniProtKB:Q96A72",
  "term_label": "Unknown molecular function"
}